condensed nuclear chromosome [GO:0000794] (cellular component) Relationships: is a type of GO:0000228; is a type of condensed chromosome [GO:0000793] Note: Note that this term and its children can be used to annotate gene products that localize to a mitotic chromosome in an organism that undergoes a 'closed mitosis' in which the nuclear envelope does not break down during mitosis and for gene products that localize to a meiotic chromosome. Also known as: meiotic chromosome, nuclear mitotic chromosome Sources: GOC:elh Definition: A highly compacted molecule of DNA and associated proteins resulting in a cytologically distinct nuclear chromosome.